proline catabolic process to 2-oxoglutarate [GO:0019495] (biological process) Also known as: proline breakdown to 2-oxoglutarate, proline catabolic process to 2-ketoglutarate, proline catabolic process to alpha-ketoglutarate, proline catabolic process to alpha-oxoglutarate, proline catabolism to 2-ketoglutarate, proline catabolism to alpha-ketoglutarate, proline catabolism to alpha-oxoglutarate, proline degradation to 2-oxoglutarate Sources: GOC:go_curators Relationships: is a type of 2-oxoglutarate metabolic process [GO:0006103]; is a type of L-proline catabolic process [GO:0006562] Definition: The chemical reactions and pathways resulting in the breakdown of proline into other compounds, including 2-oxoglutarate.